{
  "term_id": "GO:0031941",
  "term_label": "filamentous actin",
  "gene_symbol": "PDLIM5",
  "gene": "UniProtKB:Q96HC4",
  "gene_name": "PDZ and LIM domain protein 5"
}